sperm individualization complex [GO:0070864] (CC) Definition: A cellular structure that includes cytoskeletal components and part of the cell membrane. Forms at the nuclear end of a male germline syncytium, or cyst, and translocates the over the length of the syncytium in the course of sperm individualization. Each complex contains an array of 64 investment cones, one per nucleus, that move synchronously along the spermatogenic cyst. References: PMID:10588662, PMID:9550716 Sources: GOC:sart Relationships: is a type of cellular anatomical structure [GO:0110165]